{
  "gene": "UniProtKB:Q9BRX2",
  "gene_symbol": "PELO",
  "term_label": "nonfunctional rRNA decay",
  "gene_name": "Protein pelota homolog",
  "term_id": "GO:0070651"
}